{
  "term_id": "GO:0038064",
  "gene_symbol": "OSCAR",
  "term_label": "collagen receptor activity",
  "gene_name": "Osteoclast-associated immunoglobulin-like receptor",
  "gene": "UniProtKB:Q8IYS5"
}